negative regulation of phenazine biosynthetic process [GO:1900981] (biological process) Also known as: down regulation of phenazine biosynthetic process, down-regulation of phenazine biosynthetic process, downregulation of phenazine biosynthetic process, inhibition of phenazine biosynthetic process, down regulation of acridizine biosynthesis, down regulation of acridizine biosynthetic process, down regulation of azophenylene biosynthesis, down regulation of azophenylene biosynthetic process, down regulation of dibenzo-p-diazine biosynthesis, down regulation of dibenzo-p-diazine biosynthetic process, down regulation of dibenzopyrazine biosynthesis, down regulation of dibenzopyrazine biosynthetic process, down-regulation of acridizine biosynthesis, down-regulation of acridizine biosynthetic process, down-regulation of azophenylene biosynthesis, down-regulation of azophenylene biosynthetic process, down-regulation of dibenzo-p-diazine biosynthesis, down-regulation of dibenzo-p-diazine biosynthetic process, down-regulation of dibenzopyrazine biosynthesis, down-regulation of dibenzopyrazine biosynthetic process, downregulation of acridizine biosynthesis, downregulation of acridizine biosynthetic process, downregulation of azophenylene biosynthesis, downregulation of azophenylene biosynthetic process, downregulation of dibenzo-p-diazine biosynthesis, downregulation of dibenzo-p-diazine biosynthetic process, downregulation of dibenzopyrazine biosynthesis, downregulation of dibenzopyrazine biosynthetic process, inhibition of acridizine biosynthesis, inhibition of acridizine biosynthetic process, inhibition of azophenylene biosynthesis, inhibition of azophenylene biosynthetic process, inhibition of dibenzo-p-diazine biosynthesis, inhibition of dibenzo-p-diazine biosynthetic process, inhibition of dibenzopyrazine biosynthesis, inhibition of dibenzopyrazine biosynthetic process, negative regulation of acridizine biosynthesis, negative regulation of acridizine biosynthetic process, negative regulation of azophenylene biosynthesis, negative regulation of azophenylene biosynthetic process, negative regulation of dibenzo-p-diazine biosynthesis, negative regulation of dibenzo-p-diazine biosynthetic process, negative regulation of dibenzopyrazine biosynthesis, negative regulation of dibenzopyrazine biosynthetic process Relationships: is a type of negative regulation of biosynthetic process [GO:0009890]; is a type of regulation of phenazine biosynthetic process [GO:1900980]; negatively regulates GO:0002047 Sources: GOC:TermGenie, GOC:mengo_curators Definition: Any process that stops, prevents or reduces the frequency, rate or extent of phenazine biosynthetic process.